compartment pattern specification [GO:0007386] (biological process) Definition: The regionalization process in which embryonic segments are divided into compartments that will result in differences in cell differentiation. Sources: ISBN:0879694238, http://fly.ebi.ac.uk/allied-data/lk/interactive-fly/aimain/1aahome.htm Subtypes: anterior compartment pattern formation [GO:0007387], GO:0007388 Also known as: compartment specification Relationships: is a type of GO:0009952